(3R)-3-isopropenyl-6-oxoheptanoate:CoA ligase (AMP-forming) activity [GO:0052688] (MF) Also known as: 3-isopropenyl-6-oxoheptanoyl-CoA synthetase activity Relationships: is a type of CoA-ligase activity [GO:0016405]; is a type of acid-thiol ligase activity [GO:0016878] Definition: Catalysis of the reaction: (3R)-3-isopropenyl-6-oxoheptanoate + CoA-SH + ATP = H2O + AMP + diphosphate + (3R)-3-isopropenyl-6-oxoheptanoyl-CoA. Sources: KEGG_REACTION:R06515